{
  "term_label": "Unknown biological process",
  "term_id": "UNKNOWN:0002",
  "gene": "UniProtKB:Q8IXQ3",
  "gene_name": "Uncharacterized protein C9orf40",
  "gene_symbol": "C9orf40"
}